{
  "gene_symbol": "SEH1L",
  "gene_name": "Nucleoporin SEH1",
  "gene": "UniProtKB:Q96EE3",
  "term_label": "positive regulation of TORC1 signaling",
  "term_id": "GO:1904263"
}